{
  "gene_name": "PH-interacting protein",
  "gene": "UniProtKB:Q8WWQ0",
  "term_id": "GO:0006357",
  "term_label": "regulation of transcription by RNA polymerase II",
  "gene_symbol": "PHIP"
}